outer plaque of spindle pole body [GO:0005824] (cellular component) Relationships: is a type of cellular anatomical structure [GO:0110165]; is part of spindle pole body [GO:0005816] Sources: ISBN:0879693568 Subtypes: outer plaque of mitotic spindle pole body [GO:0061499] Definition: One of three laminate structures that form the spindle pole body; the outer plaque is in the cytoplasm.